{
  "gene_symbol": "TTPA",
  "gene_name": "Alpha-tocopherol transfer protein",
  "term_id": "GO:1902936",
  "gene": "UniProtKB:P49638",
  "term_label": "phosphatidylinositol bisphosphate binding"
}